{
  "gene_name": "RNA polymerase II subunit A C-terminal domain phosphatase",
  "term_id": "GO:0008420",
  "gene_symbol": "CTDP1",
  "term_label": "RNA polymerase II CTD heptapeptide repeat phosphatase activity",
  "gene": "UniProtKB:Q9Y5B0"
}